{
  "gene": "UniProtKB:O95780",
  "term_id": "GO:0000978",
  "term_label": "RNA polymerase II cis-regulatory region sequence-specific DNA binding",
  "gene_name": "Zinc finger protein 682",
  "gene_symbol": "ZNF682"
}